{
  "term_id": "GO:0031749",
  "gene": "UniProtKB:Q96NY7",
  "gene_symbol": "CLIC6",
  "term_label": "D2 dopamine receptor binding",
  "gene_name": "Chloride intracellular channel protein 6"
}